{
  "term_label": "acrosomal vesicle",
  "gene": "UniProtKB:P38567",
  "term_id": "GO:0001669",
  "gene_symbol": "SPAM1",
  "gene_name": "Hyaluronidase PH-20"
}